{
  "gene_name": "Claudin-5",
  "term_id": "UNKNOWN:0001",
  "gene_symbol": "CLDN5",
  "gene": "UniProtKB:O00501",
  "term_label": "Unknown molecular function"
}